{
  "term_label": "G protein-coupled receptor signaling pathway",
  "gene": "UniProtKB:Q8TDT2",
  "gene_symbol": "GPR152",
  "term_id": "GO:0007186",
  "gene_name": "Probable G-protein coupled receptor 152"
}